quinone biosynthetic process [GO:1901663] (biological process) Sources: GOC:TermGenie, GOC:mb, GOC:pr Subtypes: ubiquinone biosynthetic process [GO:0006744], GO:0010236, terrequinone A biosynthetic process [GO:1900796] Relationships: is a type of ketone biosynthetic process [GO:0042181]; is a type of quinone metabolic process [GO:1901661] Definition: The chemical reactions and pathways resulting in the formation of quinone. Also known as: quinone anabolism, quinone biosynthesis, quinone formation, quinone synthesis, quinone cofactor anabolism, quinone cofactor biosynthesis, quinone cofactor biosynthetic process, quinone cofactor formation, quinone cofactor synthesis